{
  "term_label": "Unknown cellular component",
  "term_id": "UNKNOWN:0003",
  "gene_name": "Transmembrane protein 161A",
  "gene_symbol": "TMEM161A",
  "gene": "UniProtKB:Q9NX61"
}